{
  "term_label": "endoplasmic reticulum membrane",
  "gene_name": "Translocating chain-associated membrane protein 1",
  "term_id": "GO:0005789",
  "gene_symbol": "TRAM1",
  "gene": "UniProtKB:Q15629"
}